positive regulation of synoviocyte proliferation [GO:1901647] (BP) Definition: Any process that activates or increases the frequency, rate or extent of synoviocyte proliferation. Also known as: up regulation of synoviocyte proliferation, up-regulation of synoviocyte proliferation, upregulation of synoviocyte proliferation, activation of synoviocyte proliferation Sources: GOC:TermGenie Relationships: is a type of GO:0050679; is a type of GO:1901645; positively regulates synoviocyte proliferation [GO:0002941]